{
  "term_id": "GO:0016020",
  "term_label": "membrane",
  "gene_symbol": "SLC2A8",
  "gene_name": "Solute carrier family 2, facilitated glucose transporter member 8",
  "gene": "UniProtKB:Q9NY64"
}